{
  "gene": "UniProtKB:P46821",
  "term_id": "GO:0016358",
  "term_label": "dendrite development",
  "gene_symbol": "MAP1B",
  "gene_name": "Microtubule-associated protein 1B"
}